{
  "term_id": "GO:0098973",
  "term_label": "structural constituent of postsynaptic actin cytoskeleton",
  "gene_name": "POTE ankyrin domain family member F",
  "gene": "UniProtKB:A5A3E0",
  "gene_symbol": "POTEF"
}